{
  "gene_name": "Transcription factor CP2-like protein 1",
  "term_id": "GO:0005634",
  "gene_symbol": "TFCP2L1",
  "term_label": "nucleus",
  "gene": "UniProtKB:Q9NZI6"
}